sulfite oxidase activity [GO:0008482] (molecular function) Definition: Catalysis of the reaction: H2O + O2 + sulfite = H2O2 + H+ + sulfate. Relationships: is a type of oxidoreductase activity, acting on a sulfur group of donors, oxygen as acceptor [GO:0016670] Sources: RHEA:24600 Note: Note that this term has a MetaCyc pathway reference as the pathway only has a single step. Also known as: sulphite oxidase activity, sulfite:oxygen oxidoreductase activity